cell motility [GO:0048870] (biological process) Regulation: regulated by regulation of cell motility [GO:2000145]; negatively regulated by negative regulation of cell motility [GO:2000146]; positively regulated by positive regulation of cell motility [GO:2000147] Subtypes: cilium or flagellum-dependent cell motility [GO:0001539], GO:0003411, cell migration [GO:0016477], cell movement involved in somal translocation [GO:0021805], cell motility involved in cerebral cortex radial glia guided migration [GO:0021814], type IV pilus-dependent motility [GO:0043107], GO:0070358, cell swimming [GO:0071975], GO:0071976, cell motility in response to potassium ion [GO:0097230], cell motility in response to calcium ion [GO:0097231], sperm motility [GO:0097722] Relationships: is a type of cellular process [GO:0009987] Definition: Any process involved in the controlled self-propelled movement of a cell that results in translocation of the cell from one place to another. Also known as: cell locomotion, movement of a cell, cell movement Sources: GOC:dgh, GOC:dph, GOC:isa_complete, GOC:mlg